sulfate:chloride antiporter activity [GO:0160044] (molecular function) Definition: Enables the transfer of a solute or solutes from one side of a membrane to the other according to the reaction: chloride(in) + sulfate(out) = chloride(out) + sulfate(in). References: PMID:17442754 Relationships: is a type of solute:inorganic anion antiporter activity [GO:0005452]; is a type of secondary active sulfate transmembrane transporter activity [GO:0008271]; is a type of chloride transmembrane transporter activity [GO:0015108]